oxidative demethylation [GO:0070989] (biological process) Definition: The process of removing one or more methyl groups from a molecule, involving the oxidation (i.e. electron loss) of one or more atoms in the substrate. Sources: GOC:BHF, GOC:mah, GOC:rl Relationships: is a type of GO:0070988 Subtypes: oxidative RNA demethylation [GO:0035513]